{
  "term_id": "GO:0005769",
  "gene_symbol": "ATP6V0D1",
  "term_label": "early endosome",
  "gene_name": "V-type proton ATPase subunit d 1",
  "gene": "UniProtKB:P61421"
}